{
  "term_label": "plasma membrane",
  "gene_name": "Olfactory receptor 4A16",
  "term_id": "GO:0005886",
  "gene": "UniProtKB:Q8NH70",
  "gene_symbol": "OR4A16"
}